{
  "term_id": "GO:0006693",
  "gene": "UniProtKB:P52895",
  "term_label": "prostaglandin metabolic process",
  "gene_symbol": "AKR1C2",
  "gene_name": "Aldo-keto reductase family 1 member C2"
}